{
  "gene": "UniProtKB:Q8WV22",
  "gene_symbol": "NSMCE1",
  "term_label": "ubiquitin-protein transferase activity",
  "gene_name": "Non-structural maintenance of chromosomes element 1 homolog",
  "term_id": "GO:0004842"
}